{
  "term_id": "GO:0005125",
  "gene": "UniProtKB:P12643",
  "term_label": "cytokine activity",
  "gene_name": "Bone morphogenetic protein 2",
  "gene_symbol": "BMP2"
}